{
  "term_label": "sodium channel regulator activity",
  "gene_name": "Sodium channel subunit beta-4",
  "gene": "UniProtKB:Q8IWT1",
  "term_id": "GO:0017080",
  "gene_symbol": "SCN4B"
}